{
  "term_id": "GO:0016519",
  "gene_symbol": "GIPR",
  "gene": "UniProtKB:P48546",
  "gene_name": "Gastric inhibitory polypeptide receptor",
  "term_label": "gastric inhibitory peptide receptor activity"
}